{
  "term_id": "GO:0042981",
  "gene_name": "F-box only protein 11",
  "gene": "UniProtKB:Q86XK2",
  "gene_symbol": "FBXO11",
  "term_label": "regulation of apoptotic process"
}